{
  "gene": "UniProtKB:P28329",
  "term_id": "GO:0043005",
  "term_label": "neuron projection",
  "gene_symbol": "CHAT",
  "gene_name": "Choline O-acetyltransferase"
}